{
  "gene_symbol": "SPINDOC",
  "term_label": "Unknown molecular function",
  "gene": "UniProtKB:Q9BUA3",
  "term_id": "UNKNOWN:0001",
  "gene_name": "Spindlin interactor and repressor of chromatin-binding protein"
}